establishment or maintenance of epithelial cell apical/basal polarity [GO:0045197] (biological process) Relationships: is_a establishment or maintenance of apical/basal cell polarity [GO:0035088] Subtypes: establishment of epithelial cell apical/basal polarity [GO:0045198], maintenance of epithelial cell apical/basal polarity [GO:0045199] Sources: GOC:bf, GOC:mah Definition: Any cellular process that results in the specification, formation or maintenance of the apicobasal polarity of an epithelial cell.